{
  "gene_name": "Zinc finger protein ZFPM1",
  "term_id": "GO:0045944",
  "term_label": "positive regulation of transcription by RNA polymerase II",
  "gene": "UniProtKB:Q8IX07",
  "gene_symbol": "ZFPM1"
}